{
  "term_label": "cytoplasm",
  "gene_symbol": "MYO5A",
  "term_id": "GO:0005737",
  "gene_name": "Unconventional myosin-Va",
  "gene": "UniProtKB:Q9Y4I1"
}